{
  "gene_symbol": "CHRM1",
  "gene": "UniProtKB:P11229",
  "gene_name": "Muscarinic acetylcholine receptor M1",
  "term_label": "chemical synaptic transmission",
  "term_id": "GO:0007268"
}